{
  "term_label": "Unknown molecular function",
  "gene_symbol": "TMEM238",
  "term_id": "UNKNOWN:0001",
  "gene_name": "Transmembrane protein 238",
  "gene": "UniProtKB:C9JI98"
}